{
  "term_label": "antiporter activity",
  "gene": "UniProtKB:Q24JQ0",
  "gene_symbol": "TMEM241",
  "term_id": "GO:0015297",
  "gene_name": "Transmembrane protein 241"
}